{
  "gene_name": "ATPase family AAA domain-containing protein 3A",
  "term_id": "GO:0007005",
  "gene_symbol": "ATAD3A",
  "term_label": "mitochondrion organization",
  "gene": "UniProtKB:Q9NVI7"
}